{
  "gene_symbol": "LOC122513141",
  "gene_name": "RING-type domain-containing protein",
  "gene": "UniProtKB:A0A2R8Y4M4",
  "term_id": "GO:0051865",
  "term_label": "protein autoubiquitination"
}